{
  "term_label": "signal transduction",
  "gene_symbol": "BEX3",
  "gene": "UniProtKB:Q00994",
  "term_id": "GO:0007165",
  "gene_name": "Protein BEX3"
}